{
  "gene_name": "Large ribosomal subunit protein uL6",
  "term_id": "GO:0003735",
  "gene": "UniProtKB:P32969",
  "term_label": "structural constituent of ribosome",
  "gene_symbol": "RPL9P9"
}